{
  "term_id": "GO:0005886",
  "gene_name": "CD5 antigen-like",
  "gene": "UniProtKB:O43866",
  "term_label": "plasma membrane",
  "gene_symbol": "CD5L"
}